sporocarp development [GO:0030584] (BP) Definition: The process whose specific outcome is the progression of a sporocarp over time, from its formation to the mature structure. The sporocarp is a spore bearing fruiting body organ. An example of this process is found in the Fungal species Coprinopsis cinerea. Sources: GOC:mah, GOC:mtg_sensu Also known as: fruiting body development Relationships: is a type of reproductive fruiting body development [GO:0030582] Subtypes: sporocarp development involved in asexual reproduction [GO:0000905], GO:0000909